{
  "term_label": "DNA-binding transcription factor activity, RNA polymerase II-specific",
  "gene": "UniProtKB:Q9ULM2",
  "gene_symbol": "ZNF490",
  "gene_name": "Zinc finger protein 490",
  "term_id": "GO:0000981"
}